{
  "term_label": "synaptic vesicle endocytosis",
  "gene_symbol": "NLGN3",
  "gene": "UniProtKB:Q9NZ94",
  "term_id": "GO:0048488",
  "gene_name": "Neuroligin-3"
}